{
  "term_label": "D-xylose catabolic process",
  "term_id": "GO:0042843",
  "gene_symbol": "DHDH",
  "gene": "UniProtKB:Q9UQ10",
  "gene_name": "Trans-1,2-dihydrobenzene-1,2-diol dehydrogenase"
}